{
  "gene_symbol": "CCR3",
  "gene_name": "C-C chemokine receptor type 3",
  "gene": "UniProtKB:P51677",
  "term_label": "immune response",
  "term_id": "GO:0006955"
}